{
  "term_id": "GO:0150093",
  "gene": "UniProtKB:Q07954",
  "gene_symbol": "LRP1",
  "gene_name": "Prolow-density lipoprotein receptor-related protein 1",
  "term_label": "amyloid-beta clearance by transcytosis"
}